{
  "gene_name": "High mobility group nucleosome-binding domain-containing protein 5",
  "gene_symbol": "HMGN5",
  "term_id": "UNKNOWN:0001",
  "term_label": "Unknown molecular function",
  "gene": "UniProtKB:P82970"
}